{
  "gene": "UniProtKB:Q8N8Q9",
  "term_id": "GO:0016020",
  "term_label": "membrane",
  "gene_name": "Magnesium transporter NIPA2",
  "gene_symbol": "NIPA2"
}